{
  "term_label": "positive regulation of ERK1 and ERK2 cascade",
  "gene_name": "ALK and LTK ligand 1",
  "gene": "UniProtKB:Q6UXT8",
  "gene_symbol": "ALKAL1",
  "term_id": "GO:0070374"
}